calcitonin gene-related peptide binding [GO:1990407] (MF) References: PMID:10882736 Sources: GOC:bhm Also known as: CGRP polypeptide binding, calcitonin-gene-related peptide binding, calcitonin-gene-related polypeptide binding Definition: Binding to calcitonin gene-related peptide (CGRP). Relationships: is a type of GO:0097644 Note: An example of this is CALCRL in human (Q16602) in PMID:10882736 (inferred from direct assay/mutant phenotype/etc.).